specification of mesonephric proximal tubule identity [GO:0061284] (biological process) Sources: GOC:mtg_kidney_jan10 Definition: The process in which the proximal tubule of the mesonephric nephron acquires its identity. Relationships: is a type of specification of mesonephric nephron tubule identity [GO:0061282]; is a type of GO:0072082; is part of mesonephric proximal tubule morphogenesis [GO:0061276]